platelet aggregation [GO:0070527] (biological process) Definition: The adhesion of one platelet to one or more other platelets via adhesion molecules. Also known as: blood platelet aggregation, thrombocyte aggregation Sources: GOC:BHF, GOC:vk Regulation: regulated by regulation of platelet aggregation [GO:0090330]; negatively regulated by negative regulation of platelet aggregation [GO:0090331]; positively regulated by GO:1901731 Relationships: is_a homotypic cell-cell adhesion [GO:0034109]; is part of GO:0030168